{
  "gene_symbol": "RBP5",
  "term_id": "GO:0005634",
  "gene_name": "Retinol-binding protein 5",
  "term_label": "nucleus",
  "gene": "UniProtKB:P82980"
}